{
  "term_id": "GO:0000278",
  "gene": "UniProtKB:Q8NHV4",
  "gene_symbol": "NEDD1",
  "gene_name": "Protein NEDD1",
  "term_label": "mitotic cell cycle"
}